{
  "gene": "UniProtKB:Q9BUJ0",
  "gene_name": "Protein ABHD14A",
  "gene_symbol": "ABHD14A",
  "term_label": "Unknown biological process",
  "term_id": "UNKNOWN:0002"
}